exit from meiosis [GO:1990947] (biological process) Definition: Any process involved in the progression from anaphase/telophase of meiosis II to the creation of end products of meiosis, in which ploidy is reduced by half. Also known as: meiotic exit References: PMID:21389117 Relationships: is_a meiotic cell cycle phase transition [GO:0044771] Regulation: RO_0002211 by regulation of exit from meiosis [GO:0106060]; negatively regulated by negative regulation of exit from meiosis [GO:0106061]; positively regulated by positive regulation of exit from meiosis [GO:0106062]